{
  "term_id": "GO:0035091",
  "gene_symbol": "SNX14",
  "gene_name": "Sorting nexin-14",
  "term_label": "phosphatidylinositol binding",
  "gene": "UniProtKB:Q9Y5W7"
}